{
  "gene_symbol": "IZUMO1R",
  "term_label": "signaling receptor activity",
  "gene_name": "Sperm-egg fusion protein Juno",
  "gene": "UniProtKB:A6ND01",
  "term_id": "GO:0038023"
}